{
  "term_label": "Unknown biological process",
  "gene_symbol": "ICMT",
  "gene": "UniProtKB:O60725",
  "term_id": "UNKNOWN:0002",
  "gene_name": "Protein-S-isoprenylcysteine O-methyltransferase"
}